{
  "gene_name": "Alpha-2A adrenergic receptor",
  "gene_symbol": "ADRA2A",
  "term_id": "UNKNOWN:0002",
  "gene": "UniProtKB:P08913",
  "term_label": "Unknown biological process"
}